{
  "term_id": "UNKNOWN:0002",
  "gene_symbol": "A0A0G2JQZ4",
  "term_label": "Unknown biological process",
  "gene_name": "Uncharacterized protein",
  "gene": "UniProtKB:A0A0G2JQZ4"
}